{
  "gene_symbol": "SPATA45",
  "term_label": "Unknown molecular function",
  "gene": "UniProtKB:Q537H7",
  "gene_name": "Spermatogenesis-associated protein 45",
  "term_id": "UNKNOWN:0001"
}